{
  "gene": "UniProtKB:Q9UKD1",
  "gene_symbol": "GMEB2",
  "gene_name": "Glucocorticoid modulatory element-binding protein 2",
  "term_label": "regulation of transcription by RNA polymerase II",
  "term_id": "GO:0006357"
}